axis specification [GO:0009798] (BP) Relationships: is a type of GO:0007389 Also known as: axis determination Definition: The establishment, maintenance and elaboration of a pattern along a line or around a point. Subtypes: embryonic axis specification [GO:0000578], growth plate cartilage axis specification [GO:0003421], GO:0007309, adaxial/abaxial axis specification [GO:0009943], radial axis specification [GO:0009945], proximal/distal axis specification [GO:0009946], centrolateral axis specification [GO:0009947], anterior/posterior axis specification [GO:0009948], dorsal/ventral axis specification [GO:0009950], anterior/posterior axis specification, follicular epithelium [GO:0030714], establishment of anatomical structure orientation [GO:0048560], left/right axis specification [GO:0070986] Sources: GOC:dph, GOC:go_curators, GOC:isa_complete